clypeo-labral disc development [GO:0035213] (biological process) Definition: The process whose specific outcome is the progression of the clypeo-labral disc over time, from its formation to the metamorphosis to form adult structures. The clypeo-labral disc develops into the labrum, anterior cibarial plate, fish trap bristles, epistomal sclerite. Relationships: is a type of imaginal disc development [GO:0007444] Also known as: development of structures derived from the clypeo-labral disc Sources: GOC:bf, ISBN:0879694238